{
  "gene": "UniProtKB:Q96CT2",
  "term_id": "GO:0043161",
  "term_label": "proteasome-mediated ubiquitin-dependent protein catabolic process",
  "gene_name": "Kelch-like protein 29",
  "gene_symbol": "KLHL29"
}